{
  "gene_name": "ADP-ribosylation factor-like protein 2",
  "gene_symbol": "ARL2",
  "term_label": "microtubule cytoskeleton",
  "gene": "UniProtKB:P36404",
  "term_id": "GO:0015630"
}